{
  "term_label": "negative regulation of insulin receptor signaling pathway",
  "gene_symbol": "TNS2",
  "term_id": "GO:0046627",
  "gene": "UniProtKB:Q63HR2",
  "gene_name": "Tensin-2"
}